intracellular borate homeostasis [GO:0160070] (biological process) Relationships: is a type of intracellular chemical homeostasis [GO:0055082]; is a type of GO:0098771 Definition: A homeostatic process involved in the maintenance of a steady state level of tetrahydroxoborate within a cell. References: PMID:15525507 Also known as: intracellular boron homeostasis, intracellular tetrahydroxoborate homeostasis